regulation of thyroid hormone receptor signaling pathway [GO:0002155] (biological process) Relationships: is a type of regulation of intracellular signal transduction [GO:1902531]; regulates thyroid hormone receptor signaling pathway [GO:0002154] Subtypes: negative regulation of thyroid hormone receptor signaling pathway [GO:0002156], GO:0002157 Definition: Any process that modulates the frequency, rate or extent of a thyroid hormone mediated signaling pathway. Also known as: regulation of thyroid hormone mediated signaling pathway, regulation of thyroid hormone mediated signalling pathway Sources: GOC:hjd